{
  "term_label": "ubiquitin protein ligase activity",
  "gene_symbol": "RNF145",
  "gene": "UniProtKB:Q96MT1",
  "term_id": "GO:0061630",
  "gene_name": "RING finger protein 145"
}